positive regulation of cilium-dependent cell motility [GO:2000155] (biological process) Definition: Any process that activates or increases the frequency, rate or extent of cilium-dependent cell motility. Sources: GOC:cilia, GOC:jl Also known as: positive regulation of ciliary cell motility Relationships: is a type of regulation of cilium-dependent cell motility [GO:1902019]; is_a positive regulation of cell motility [GO:2000147]; positively regulates cilium-dependent cell motility [GO:0060285] Subtypes: positive regulation of flagellated sperm motility [GO:1902093]